{
  "gene_name": "Mast_stem cell growth factor receptor Kit",
  "term_id": "GO:0002244",
  "gene_symbol": "KIT",
  "term_label": "hematopoietic progenitor cell differentiation",
  "gene": "UniProtKB:P10721"
}